{
  "term_label": "nucleus",
  "gene": "UniProtKB:Q96NZ1",
  "term_id": "GO:0005634",
  "gene_symbol": "FOXN4",
  "gene_name": "Forkhead box protein N4"
}